glial cell differentiation involved in amphid sensory organ development [GO:0003398] (biological process) Definition: The process in which a relatively unspecialized cell acquires the specialized features of a glial cell of the amphid sensory organ. Sources: GOC:ascb_2009, GOC:dph, GOC:tb Relationships: is a type of glial cell differentiation [GO:0010001]; is part of amphid sensory organ development [GO:0003386]